{
  "gene_symbol": "CD46",
  "gene": "UniProtKB:P15529",
  "gene_name": "Membrane cofactor protein",
  "term_id": "GO:0002456",
  "term_label": "T cell mediated immunity"
}